{
  "gene_name": "Junction plakoglobin",
  "gene_symbol": "JUP",
  "term_id": "GO:0045296",
  "gene": "UniProtKB:P14923",
  "term_label": "cadherin binding"
}